{
  "gene_name": "Arf-GAP with dual PH domain-containing protein 1",
  "gene_symbol": "ADAP1",
  "term_label": "GTPase activator activity",
  "gene": "UniProtKB:O75689",
  "term_id": "GO:0005096"
}